{
  "gene": "UniProtKB:Q9Y289",
  "term_label": "pantothenate transmembrane transport",
  "gene_name": "Sodium-dependent multivitamin transporter",
  "gene_symbol": "SLC5A6",
  "term_id": "GO:0015887"
}